{
  "gene": "UniProtKB:P41219",
  "gene_symbol": "PRPH",
  "term_label": "plasma membrane",
  "term_id": "GO:0005886",
  "gene_name": "Peripherin"
}